{
  "term_label": "regulation of lymphocyte migration",
  "term_id": "GO:2000401",
  "gene_symbol": "STK10",
  "gene": "UniProtKB:O94804",
  "gene_name": "Serine_threonine-protein kinase 10"
}